{
  "term_id": "GO:0005886",
  "gene_name": "Lens fiber major intrinsic protein",
  "gene": "UniProtKB:P30301",
  "gene_symbol": "MIP",
  "term_label": "plasma membrane"
}